mitotic cell cycle phase [GO:0098763] (biological process) Note: This term should not be used for direct annotation. If you are trying to make an annotation to x phase, it is likely that the correct annotation should be to 'regulation of x/y phase transition' or to a process which occurs during the reported phase (e.g. mitotic DNA replication for mitotic S-phase). To capture the phase when a specific location or process is observed, the phase term can be used in an annotation extension (PMID:24885854) applied to a cellular component term (with the relation exists_during) or a biological process term (with the relation happens_during). Relationships: is a type of cell cycle phase [GO:0022403]; happens during GO:0000278 Definition: One of the distinct periods or stages into which the mitotic cell cycle is divided. Each phase is characterized by the occurrence of specific biochemical and morphological events. Sources: GOC:dos Subtypes: mitotic M phase [GO:0000087], mitotic interphase [GO:0051329]